{
  "term_label": "negative regulation of execution phase of apoptosis",
  "term_id": "GO:1900118",
  "gene": "UniProtKB:P0CJ75",
  "gene_symbol": "MTRNR2L8",
  "gene_name": "Humanin-like 8"
}